{
  "gene_symbol": "CFAP418",
  "term_label": "ciliary base",
  "gene_name": "Cilia- and flagella-associated protein 418",
  "term_id": "GO:0097546",
  "gene": "UniProtKB:Q96NL8"
}